activin receptor antagonist activity [GO:0038102] (MF) References: PMID:15062104 Sources: GOC:signaling Note: This term refers to inhibition of a member of the activin receptor family; activin receptors bind to multiple ligands including activin and nodal. Relationships: is a type of receptor antagonist activity [GO:0048019]; is part of negative regulation of activin receptor signaling pathway [GO:0032926] Definition: Interacting with an activin receptor complex to reduce the action of another ligand, the agonist. A receptor antagonist does not initiate signaling upon binding to a receptor, but instead blocks an agonist from binding to the receptor.